{
  "term_id": "GO:0042127",
  "term_label": "regulation of cell population proliferation",
  "gene_symbol": "STAT1",
  "gene_name": "Signal transducer and activator of transcription 1-alpha_beta",
  "gene": "UniProtKB:P42224"
}